establishment of protein localization to endoplasmic reticulum membrane [GO:0097051] (biological process) Also known as: establishment of protein localisation in endoplasmic reticulum membrane, establishment of protein localization in endoplasmic reticulum membrane References: PMID:9388185 Sources: GOC:rb Relationships: is a type of GO:0072599; is a type of establishment of protein localization to membrane [GO:0090150] Definition: The directed movement of a protein to a specific location in the endoplasmic reticulum membrane.